amine-lyase activity [GO:0016843] (molecular function) Subtypes: GO:0036381, 3-ketovalidoxylamine C-N-lyase activity [GO:0047566], mimosinase activity [GO:0050101] Relationships: is a type of GO:0016840 Sources: GOC:krc Definition: Catalysis of the release of amines by the cleavage of a carbon-nitrogen bond or the reverse reaction with an amine as a substrate.